{
  "gene_name": "Late cornified envelope protein 6A",
  "term_id": "UNKNOWN:0003",
  "gene_symbol": "LCE6A",
  "term_label": "Unknown cellular component",
  "gene": "UniProtKB:A0A183"
}